{
  "term_label": "synaptic vesicle membrane organization",
  "gene_symbol": "AP3D1",
  "term_id": "GO:0048499",
  "gene_name": "AP-3 complex subunit delta-1",
  "gene": "UniProtKB:O14617"
}